{
  "gene_symbol": "RNF144A",
  "gene_name": "E3 ubiquitin-protein ligase RNF144A",
  "term_label": "Golgi apparatus",
  "term_id": "GO:0005794",
  "gene": "UniProtKB:P50876"
}